hemicellulose network [GO:0048223] (cellular component) Definition: Network composed of hemicelluloses; members of a class of plant cell wall polysaccharide that cannot be extracted from the wall by hot water or chelating agents, but can be extracted by aqueous alkali. Includes xylan, glucuronoxylan, arabinoxylan, arabinogalactan II, glucomannan, xyloglucan and galactomannan. Sources: DOI:10.1016/j.foodchem.2008.11.065, GOC:jid Relationships: is a type of cellular anatomical structure [GO:0110165]; is part of primary cell wall [GO:0009530]; BFO_0000050 GO:0009531